{
  "term_label": "Unknown cellular component",
  "gene_name": "Transmembrane protein 244",
  "gene_symbol": "TMEM244",
  "gene": "UniProtKB:Q5VVB8",
  "term_id": "UNKNOWN:0003"
}